dihydrolipoyl dehydrogenase (NADH) activity [GO:0004148] (molecular function) Sources: RHEA:15045 Also known as: LDP-Glc activity, LDP-Val activity, E3 component of alpha-ketoacid dehydrogenase complexes activity, L-protein activity, dehydrolipoate dehydrogenase activity, diaphorase activity, dihydrolipoamide dehydrogenase activity, dihydrolipoamide reduction, dihydrolipoamide:NAD+ oxidoreductase, dihydrolipoic dehydrogenase activity, dihydrolipoylprotein reduction, dihydrothioctic dehydrogenase activity, glycine-cleavage system L-protein activity, lipoamide dehydrogenase (NADH) activity, lipoamide oxidoreductase (NADH) activity, lipoamide reductase (NADH) activity, lipoamide reductase activity, lipoate dehydrogenase activity, lipoic acid dehydrogenase activity, lipoyl dehydrogenase activity, protein-6-N-(dihydrolipoyl)lysine:NAD+ oxidoreductase, protein-N6-(dihydrolipoyl)lysine:NAD+ oxidoreductase Relationships: is a type of oxidoreductase activity, acting on a sulfur group of donors, NAD(P) as acceptor [GO:0016668] Definition: Catalysis of the reaction: N(6)-[(R)-dihydrolipoyl]-L-lysyl-[protein] + NAD+ = N(6)-[(R)-lipoyl]-L-lysyl-[protein] + NADH + H+.